{
  "term_label": "Unknown molecular function",
  "gene": "UniProtKB:P28066",
  "gene_name": "Proteasome subunit alpha type-5",
  "term_id": "UNKNOWN:0001",
  "gene_symbol": "PSMA5"
}